protein autoubiquitination [GO:0051865] (biological process) Definition: The ubiquitination by a protein of one or more of its own amino acid residues, or residues on an identical protein. Ubiquitination occurs on the lysine residue by formation of an isopeptide crosslink. Sources: GOC:ai Also known as: protein auto-ubiquitination, protein auto-ubiquitinylation, protein autoubiquitinylation, protein self-ubiquitination, protein self-ubiquitinylation Relationships: is a type of protein ubiquitination [GO:0016567] Regulation: regulated by regulation of protein autoubiquitination [GO:1902498]; positively regulated by positive regulation of protein autoubiquitination [GO:1902499]; negatively regulated by negative regulation of protein autoubiquitination [GO:1905524]